ethanolamine-phosphate phospho-lyase activity [GO:0050459] (molecular function) Also known as: amino alcohol O-phosphate phospholyase activity, O-phosphoethanolamine-phospholyase activity, O-phosphorylethanol-amine phospho-lyase activity, ethanolamine-phosphate phospho-lyase (deaminating), ethanolamine-phosphate phospho-lyase (deaminating; acetaldehyde-forming) Sources: EC:4.2.3.2, RHEA:17889 Definition: Catalysis of the reaction: H2O + phosphoethanolamine = acetaldehyde + NH4 + phosphate. Relationships: is a type of GO:0016838